{
  "gene": "UniProtKB:O43542",
  "term_id": "GO:0000400",
  "term_label": "four-way junction DNA binding",
  "gene_name": "DNA repair protein XRCC3",
  "gene_symbol": "XRCC3"
}